{
  "gene": "UniProtKB:P08237",
  "gene_symbol": "PFKM",
  "gene_name": "ATP-dependent 6-phosphofructokinase, muscle type",
  "term_id": "GO:0005945",
  "term_label": "6-phosphofructokinase complex"
}